mercury (II) reductase (NADP+) activity [GO:0016152] (molecular function) Also known as: Hg:NADP+ oxidoreductase activity, mer A, mercurate(II) reductase activity, mercuric ion reductase activity, mercuric reductase activity, mercury reductase activity, mercury(II) reductase activity, reduced NADP:mercuric ion oxidoreductase activity Definition: Catalysis of the reaction: H+ + Hg + NADP+ = Hg2+ + NADPH. Sources: RHEA:23856 Relationships: is a type of oxidoreductase activity, acting on metal ions, NAD or NADP as acceptor [GO:0016723]